UDP-galactose:N-glycan beta-1,3-galactosyltransferase activity [GO:0010488] (molecular function) References: PMID:17630273 Definition: Catalysis of the reaction: UDP-galactose + N-glycan = galactose-beta-1,3-N-glycan + UDP. Relationships: is a type of GO:0035250